{
  "term_id": "GO:0005783",
  "gene_symbol": "SERP2",
  "gene": "UniProtKB:Q8N6R1",
  "gene_name": "Stress-associated endoplasmic reticulum protein 2",
  "term_label": "endoplasmic reticulum"
}